{
  "gene": "UniProtKB:P50150",
  "gene_name": "Guanine nucleotide-binding protein G(I)_G(S)_G(O) subunit gamma-4",
  "term_id": "GO:0031681",
  "term_label": "G-protein beta-subunit binding",
  "gene_symbol": "GNG4"
}